{
  "term_id": "UNKNOWN:0002",
  "gene_name": "MaFF-interacting protein",
  "gene_symbol": "MAFIP",
  "gene": "UniProtKB:Q8WZ33",
  "term_label": "Unknown biological process"
}